{
  "term_label": "cilium assembly",
  "gene_symbol": "CCDC66",
  "gene_name": "Coiled-coil domain-containing protein 66",
  "gene": "UniProtKB:A2RUB6",
  "term_id": "GO:0060271"
}